basolateral part of cell [GO:1990794] (cellular component) Relationships: is a type of cellular anatomical structure [GO:0110165]; is part of basal part of cell [GO:0045178]; is part of GO:0097574 Definition: The region of a cell situated by the cell sides which interface adjacent cells and near the base. Often used in reference to animal polarized epithelial cells. References: PMID:18495799